{
  "term_label": "error-prone translesion synthesis",
  "gene_symbol": "POLK",
  "term_id": "GO:0042276",
  "gene": "UniProtKB:Q9UBT6",
  "gene_name": "DNA polymerase kappa"
}